{
  "gene_symbol": "SYNGR1",
  "gene_name": "Synaptogyrin-1",
  "gene": "UniProtKB:O43759",
  "term_label": "Unknown molecular function",
  "term_id": "UNKNOWN:0001"
}